{
  "gene": "UniProtKB:Q92540",
  "term_label": "telomeric DNA binding",
  "gene_symbol": "SMG7",
  "gene_name": "Nonsense-mediated mRNA decay factor SMG7",
  "term_id": "GO:0042162"
}